{
  "term_label": "endoplasmic reticulum membrane",
  "gene_name": "Glucose-6-phosphate exchanger SLC37A4",
  "term_id": "GO:0005789",
  "gene_symbol": "SLC37A4",
  "gene": "UniProtKB:O43826"
}